regulation of cardiac muscle cell apoptotic process [GO:0010665] (biological process) Sources: GOC:dph, GOC:mtg_apoptosis, GOC:tb Relationships: is a type of regulation of striated muscle cell apoptotic process [GO:0010662]; regulates cardiac muscle cell apoptotic process [GO:0010659] Also known as: regulation of cardiac muscle cell apoptosis Definition: Any process that modulates the rate or extent of cardiac cell apoptotic process, a form of programmed cell death induced by external or internal signals that trigger the activity of proteolytic caspases whose actions dismantle a cardiac muscle cell and result in its death. Subtypes: GO:0010666, negative regulation of cardiac muscle cell apoptotic process [GO:0010667]